{
  "gene_symbol": "PGM2",
  "gene": "UniProtKB:Q96G03",
  "gene_name": "Phosphopentomutase",
  "term_id": "GO:0008973",
  "term_label": "phosphopentomutase activity"
}